{
  "term_label": "negative regulation of transcription by RNA polymerase II",
  "term_id": "GO:0000122",
  "gene_symbol": "NR1D2",
  "gene": "UniProtKB:Q14995",
  "gene_name": "Nuclear receptor subfamily 1 group D member 2"
}